{
  "gene_name": "Ceramide-1-phosphate transfer protein",
  "gene": "UniProtKB:Q5TA50",
  "term_label": "ceramide 1-phosphate binding",
  "gene_symbol": "CPTP",
  "term_id": "GO:1902387"
}